{
  "gene": "UniProtKB:P56693",
  "gene_symbol": "SOX10",
  "term_label": "peripheral nervous system development",
  "gene_name": "Transcription factor SOX-10",
  "term_id": "GO:0007422"
}